{
  "gene": "UniProtKB:P31321",
  "term_id": "GO:0030552",
  "gene_name": "cAMP-dependent protein kinase type I-beta regulatory subunit",
  "gene_symbol": "PRKAR1B",
  "term_label": "cAMP binding"
}